tRNA (guanine(27)-N2)-dimethyltransferase activity [GO:0160248] (molecular function) Relationships: is a type of GO:0008170; is a type of tRNA (guanine) methyltransferase activity [GO:0016423] References: PMID:39786990, PMID:39786998 Definition: Catalysis of the reaction: guanosine(27) in tRNA + 2 S-adenosyl-L-methionine = 2 H+ + N(2)-dimethylguanosine(27) in tRNA + 2 S-adenosyl-L-homocysteine.